{
  "gene_symbol": "TCP11",
  "gene": "UniProtKB:Q8WWU5",
  "gene_name": "T-complex protein 11 homolog",
  "term_label": "regulation of sperm capacitation",
  "term_id": "GO:1902490"
}